WASH complex [GO:0071203] (cellular component) References: PMID:19922875 Sources: GOC:sp Relationships: is a type of protein-containing complex [GO:0032991]; is part of cytoplasm [GO:0005737] Definition: A protein complex that localizes at the surface of endosomes, where it recruits and activates the Arp2/3 complex to induce actin polymerization. In human, the WASH complex is composed of F-actin-capping protein subunits alpha and beta, WASH1, FAM21, KIAA1033, KIAA0196 and CCDC53.